{
  "term_label": "ketohexokinase activity",
  "gene_name": "Ketohexokinase",
  "gene": "UniProtKB:P50053",
  "term_id": "GO:0004454",
  "gene_symbol": "KHK"
}